{
  "gene_symbol": "TAF11L12",
  "gene_name": "TATA-box-binding protein-associated factor 11-like protein 12",
  "term_id": "GO:0016251",
  "term_label": "RNA polymerase II general transcription initiation factor activity",
  "gene": "UniProtKB:A0A1W2PPW3"
}